TNFSF11 binding [GO:0038057] (molecular function) Definition: Binding to tumor necrosis factor ligand superfamily member 11 (TNFSF11), a member of the tumor necrosis factor (TNF) cytokine family. Sources: GOC:cjm Relationships: is a type of tumor necrosis factor binding [GO:0043120] Also known as: CD254 binding, ODF binding, OPGL binding, RANKL binding, TNF-related activation-induced cytokine binding, TRANCE binding, osteoclast differentiation factor binding, osteoprotegerin ligand binding, receptor activator of nuclear factor kappa-B ligand binding, tumor necrosis factor (ligand) superfamily member 11 binding, tumor necrosis factor ligand superfamily member 11 binding, tumor necrosis factor superfamily member 11 binding